protein targeting to peroxisome [GO:0006625] (biological process) Sources: GOC:ai Relationships: is a type of GO:0006605; is a type of establishment of protein localization to peroxisome [GO:0072663] Definition: The process of directing proteins towards the peroxisome, usually using signals contained within the protein. Also known as: protein-peroxisome targeting